{
  "gene_name": "Trypsin-3",
  "gene": "UniProtKB:P35030",
  "gene_symbol": "PRSS3",
  "term_label": "extracellular space",
  "term_id": "GO:0005615"
}